oral apparatus organization [GO:0032122] (biological process) Relationships: is a type of cellular component organization [GO:0016043] References: PMID:10503189, PMID:6414830 Definition: A process that is carried out at the cellular level which results in the assembly, arrangement of constituent parts, or disassembly of the oral apparatus. The oral apparatus is a funnel-like structure used by the cell to collect food and channel it to the cytostome, characteristic of ciliate protozoans. Also known as: oral apparatus organisation, oral apparatus morphogenesis, oral apparatus organization and biogenesis, stomatogenesis